{
  "gene_symbol": "YIPF5",
  "gene": "UniProtKB:Q969M3",
  "gene_name": "Protein YIPF5",
  "term_label": "trans-Golgi network",
  "term_id": "GO:0005802"
}